{
  "term_id": "GO:0016477",
  "term_label": "cell migration",
  "gene_name": "Protein WWC2",
  "gene_symbol": "WWC2",
  "gene": "UniProtKB:Q6AWC2"
}